{
  "term_id": "GO:0033344",
  "gene": "UniProtKB:P35610",
  "gene_name": "Sterol O-acyltransferase 1",
  "term_label": "cholesterol efflux",
  "gene_symbol": "SOAT1"
}